{
  "gene_symbol": "B4GALNT3",
  "gene": "UniProtKB:Q6L9W6",
  "term_label": "Unknown biological process",
  "gene_name": "Beta-1,4-N-acetylgalactosaminyltransferase 3",
  "term_id": "UNKNOWN:0002"
}